negative regulation of protection from non-homologous end joining at telomere [GO:1905765] (biological process) References: PMID:14690602 Sources: GOC:BHF, GOC:BHF_telomere, GOC:TermGenie, GOC:nc, GO_REF:0000058 Definition: Any process that stops, prevents or reduces the frequency, rate or extent of protection from non-homologous end joining at telomere. Also known as: down regulation of protection from NHEJ-mediated telomere fusion, down regulation of protection from non-homologous end joining at telomere, down-regulation of protection from NHEJ-mediated telomere fusion, down-regulation of protection from non-homologous end joining at telomere, downregulation of protection from NHEJ-mediated telomere fusion, downregulation of protection from non-homologous end joining at telomere, negative regulation of protection from NHEJ-mediated telomere fusion, inhibition of protection from NHEJ-mediated telomere fusion, inhibition of protection from non-homologous end joining at telomere Relationships: is a type of negative regulation of telomere capping [GO:1904354]; is_a negative regulation of telomere maintenance in response to DNA damage [GO:1904506]; is a type of regulation of protection from non-homologous end joining at telomere [GO:1905764]; negatively regulates protection from non-homologous end joining at telomere [GO:0031848]